{
  "term_label": "phosphatidylglycerol metabolic process",
  "term_id": "GO:0046471",
  "gene_name": "Phospholipase A2 group V",
  "gene_symbol": "PLA2G5",
  "gene": "UniProtKB:P39877"
}